tricuspid valve morphogenesis [GO:0003186] (biological process) Sources: GOC:mtg_heart Definition: The process in which the structure of the tricuspid valve is generated and organized. Relationships: is a type of atrioventricular valve morphogenesis [GO:0003181]; is part of GO:0003175